{
  "term_label": "Unknown cellular component",
  "term_id": "UNKNOWN:0003",
  "gene_symbol": "TAC3",
  "gene": "UniProtKB:Q9UHF0",
  "gene_name": "Tachykinin-3"
}